{
  "term_label": "potassium channel regulator activity",
  "term_id": "GO:0015459",
  "gene": "UniProtKB:P42658",
  "gene_symbol": "DPP6",
  "gene_name": "Dipeptidyl aminopeptidase-like protein 6"
}